{
  "term_id": "GO:0042110",
  "term_label": "T cell activation",
  "gene": "UniProtKB:O95267",
  "gene_name": "RAS guanyl-releasing protein 1",
  "gene_symbol": "RASGRP1"
}